glucosylglycerol transmembrane transport [GO:0051475] (biological process) Sources: GOC:ai Also known as: glucosylglycerol transport Relationships: is a type of polyol transmembrane transport [GO:0015791]; is a type of carbohydrate transmembrane transport [GO:0034219]; is a type of glycoside transport [GO:1901656] Definition: The directed movement of glucosylglycerol, alpha-D-glucopyranosyl-alpha-(1,2)-glycerol, across a membrane.